response to mineralocorticoid [GO:0051385] (biological process) Subtypes: response to corticosterone [GO:0051412], GO:0071389, response to 11-deoxycorticosterone [GO:1903496], response to aldosterone [GO:1904044] Also known as: response to mineralocorticoid stimulus Relationships: is a type of response to corticosteroid [GO:0031960] Definition: Any process that results in a change in state or activity of a cell or an organism (in terms of movement, secretion, enzyme production, gene expression, etc.) as a result of a mineralocorticoid stimulus. Mineralocorticoids are hormonal C21 corticosteroids synthesized from cholesterol and characterized by their similarity to aldosterone. Mineralocorticoids act primarily on water and electrolyte balance. References: PMID:9884123 Sources: GOC:ai